{
  "term_label": "ubiquitin binding",
  "gene_symbol": "FBXW7",
  "term_id": "GO:0043130",
  "gene": "UniProtKB:Q969H0",
  "gene_name": "F-box_WD repeat-containing protein 7"
}